{
  "gene_symbol": "SLC1A1",
  "term_label": "L-glutamate transmembrane transport",
  "gene": "UniProtKB:P43005",
  "term_id": "GO:0015813",
  "gene_name": "Excitatory amino acid transporter 3"
}